{
  "gene_name": "Dynein axonemal heavy chain 1",
  "term_label": "minus-end-directed microtubule motor activity",
  "gene": "UniProtKB:Q9P2D7",
  "gene_symbol": "DNAH1",
  "term_id": "GO:0008569"
}